biological process involved in interaction with host [GO:0051701] (biological process) Subtypes: symbiont-mediated killing of host cell [GO:0001907], GO:0030581, exit from host cell [GO:0035891], migration in host [GO:0044001], acquisition of nutrients from host [GO:0044002], GO:0044003, adhesion of symbiont to host [GO:0044406], symbiont entry into host [GO:0044409], translocation of molecules into host [GO:0044417], response to host [GO:0075136] Also known as: interaction with host, growth of symbiont in host, growth of symbiont in host cell, growth of symbiont in host organelle, growth of symbiont in host vacuole Sources: GOC:cc Definition: An interaction between two organisms living together in more or less intimate association. The term host is used for the larger (macro) of the two members of a symbiosis; the various forms of symbiosis include parasitism, commensalism and mutualism. Relationships: is a type of biological process involved in symbiotic interaction [GO:0044403]